chloroplast disassembly [GO:1904821] (biological process) Relationships: is_a chloroplast organization [GO:0009658]; is a type of organelle disassembly [GO:1903008] Also known as: chloroplast degradation Definition: The disaggregation of a chloroplast into its constituent components. References: PMID:26494759 Sources: GOC:TermGenie, GO_REF:0000079 Note: The disaggregation of a chloroplast into its constituent components.